organofluorine metabolic process [GO:0090346] (biological process) Sources: GOC:BHF Definition: The chemical reactions and pathways involving organofluorine compounds, as carried out by individual cells. Subtypes: methyl fluoride metabolic process [GO:0018929] Relationships: is a type of organohalogen metabolic process [GO:0090345] Regulation: negatively regulated by negative regulation of organofluorine metabolic process [GO:0090350]